{
  "term_id": "GO:0000137",
  "term_label": "Golgi cis cisterna",
  "gene_symbol": "GOLGA8O",
  "gene": "UniProtKB:A6NCC3",
  "gene_name": "Golgin subfamily A member 8O"
}